{
  "term_label": "nucleus",
  "gene_name": "Iroquois-class homeodomain protein IRX-6",
  "term_id": "GO:0005634",
  "gene": "UniProtKB:P78412",
  "gene_symbol": "IRX6"
}